{
  "gene_name": "Anion exchange protein 2",
  "term_label": "plasma membrane",
  "gene_symbol": "SLC4A2",
  "gene": "UniProtKB:P04920",
  "term_id": "GO:0005886"
}